nuclear outer membrane [GO:0005640] (cellular component) Also known as: nucleus outer envelope, perinuclear membrane Sources: ISBN:0198547684 Definition: The outer, i.e. cytoplasm-facing, lipid bilayer of the nuclear envelope; continuous with the endoplasmic reticulum of the cell and sometimes studded with ribosomes. Relationships: is a type of GO:0031965; is a type of organelle outer membrane [GO:0031968]; is part of nuclear outer membrane-endoplasmic reticulum membrane network [GO:0042175]